{
  "gene_name": "Lethal(3)malignant brain tumor-like protein 3",
  "gene": "UniProtKB:Q96JM7",
  "term_id": "GO:0042393",
  "gene_symbol": "L3MBTL3",
  "term_label": "histone binding"
}